{
  "term_id": "GO:0019789",
  "term_label": "SUMO transferase activity",
  "gene": "UniProtKB:Q99666",
  "gene_name": "RANBP2-like and GRIP domain-containing protein 5_6",
  "gene_symbol": "RGPD5"
}